{
  "gene_symbol": "C5AR1",
  "gene_name": "C5a anaphylatoxin chemotactic receptor 1",
  "term_label": "positive regulation of cytosolic calcium ion concentration",
  "gene": "UniProtKB:P21730",
  "term_id": "GO:0007204"
}